{
  "term_id": "GO:0006357",
  "gene_name": "Bromodomain testis-specific protein",
  "term_label": "regulation of transcription by RNA polymerase II",
  "gene_symbol": "BRDT",
  "gene": "UniProtKB:Q58F21"
}